{
  "term_label": "phytol metabolic process",
  "gene_name": "Peroxisomal trans-2-enoyl-CoA reductase",
  "term_id": "GO:0033306",
  "gene_symbol": "PECR",
  "gene": "UniProtKB:Q9BY49"
}